{
  "gene_symbol": "FAM178B",
  "gene": "UniProtKB:Q8IXR5",
  "term_label": "Unknown cellular component",
  "gene_name": "Protein FAM178B",
  "term_id": "UNKNOWN:0003"
}